{
  "gene_name": "Voltage-dependent calcium channel gamma-3 subunit",
  "term_label": "transmission of nerve impulse",
  "term_id": "GO:0019226",
  "gene_symbol": "CACNG3",
  "gene": "UniProtKB:O60359"
}